{
  "gene_symbol": "PGR",
  "term_id": "GO:0006357",
  "gene": "UniProtKB:P06401",
  "term_label": "regulation of transcription by RNA polymerase II",
  "gene_name": "Progesterone receptor"
}